{
  "term_id": "GO:0071546",
  "gene_symbol": "ANKRD34C",
  "gene_name": "Ankyrin repeat domain-containing protein 34C",
  "gene": "UniProtKB:P0C6C1",
  "term_label": "pi-body"
}